{
  "gene": "UniProtKB:Q8WWN8",
  "gene_symbol": "ARAP3",
  "term_id": "GO:0005737",
  "term_label": "cytoplasm",
  "gene_name": "Arf-GAP with Rho-GAP domain, ANK repeat and PH domain-containing protein 3"
}